spore-bearing structure development [GO:0075259] (biological process) Also known as: sporangium development, fruiting structure development, sporophore development, spore-bearing organ development Relationships: is a type of reproductive structure development [GO:0048608] Subtypes: GO:0030582, sporangium development [GO:0043582], GO:0070787, oogonium development [GO:0075263], zygosporangium development [GO:0075271], telium development [GO:0075275], uredinium development [GO:0075279], basidium development [GO:0075313], ascus development [GO:0075317] Sources: GOC:di, GOC:mah, GOC:mcc, GOC:pamgo_curators Regulation: regulated by regulation of spore-bearing organ development [GO:0075260]; positively regulated by positive regulation of spore-bearing organ development [GO:0075261]; negatively regulated by negative regulation of spore-bearing organ development [GO:0075262] Definition: The process whose specific outcome is the progression of a spore-bearing structure over time, from its formation to the mature structure. A spore-bearing structure is an anatomical structure that produces new spores.